{
  "gene": "UniProtKB:Q9H8Y8",
  "gene_name": "Golgi reassembly-stacking protein 2",
  "term_label": "Unknown molecular function",
  "term_id": "UNKNOWN:0001",
  "gene_symbol": "GORASP2"
}